trioxoheptanoate hydrolase activity [GO:0018772] (molecular function) Definition: Catalysis of the reaction: 2,4,6-trioxoheptanoate + H2O = acetylpyruvate + acetate. Sources: MetaCyc:R306-RXN, UM-BBD_reactionID:r0094 Relationships: is a type of hydrolase activity, acting on acid carbon-carbon bonds, in ketonic substances [GO:0016823]